branched 1,3-beta-D-glucan synthase activity [GO:0140752] (molecular function) Relationships: is a type of 1,3-beta-D-glucan synthase activity [GO:0003843] Definition: Catalysis of the reaction: UDP-glucose + [(1->3)-beta-D-glucosyl](n) = UDP + a branched [(1->3)-beta-D-glucosyl](n+1). References: PMID:34959732